{
  "gene_name": "Olfactory receptor 1Q1",
  "term_id": "GO:0005886",
  "term_label": "plasma membrane",
  "gene": "UniProtKB:Q15612",
  "gene_symbol": "OR1Q1"
}